membrane depolarization during SA node cell action potential [GO:0086046] (biological process) Relationships: is_a GO:0086012; is part of SA node cell action potential [GO:0086015] Sources: GOC:BHF, GOC:mtg_cardiac_conduct_nov11 Definition: The process in which SA node cardiac muscle cell membrane potential changes in the depolarizing direction from the negative resting potential towards the positive membrane potential that will be the peak of the action potential. Also known as: membrane depolarization involved in regulation of SA node cardiac muscle cell action potential, membrane depolarization involved in regulation of SAN cardiac muscle cell action potential, membrane depolarization involved in regulation of sinoatrial node cardiac muscle cell action potential, membrane depolarization involved in regulation of sinus node cardiac muscle cell action potential